{
  "gene_symbol": "B3GALT1",
  "term_label": "N-acetyl-beta-D-glucosaminide beta-(1,3)-galactosyltransferase activity",
  "gene": "UniProtKB:Q9Y5Z6",
  "term_id": "GO:0008499",
  "gene_name": "Beta-1,3-galactosyltransferase 1"
}